{
  "gene_symbol": "FGF20",
  "term_id": "GO:0005615",
  "term_label": "extracellular space",
  "gene": "UniProtKB:Q9NP95",
  "gene_name": "Fibroblast growth factor 20"
}